{
  "gene_name": "Cysteinyl leukotriene receptor 2",
  "gene_symbol": "CYSLTR2",
  "term_id": "GO:0004966",
  "term_label": "galanin receptor activity",
  "gene": "UniProtKB:Q9NS75"
}